{
  "gene_name": "Phosphatidylinositol 3-kinase C2 domain-containing subunit gamma",
  "term_id": "GO:0016477",
  "gene": "UniProtKB:O75747",
  "term_label": "cell migration",
  "gene_symbol": "PIK3C2G"
}